{
  "term_id": "UNKNOWN:0003",
  "term_label": "Unknown cellular component",
  "gene_symbol": "RNF225",
  "gene_name": "RING finger protein 225",
  "gene": "UniProtKB:M0QZC1"
}